{
  "term_label": "chromatin organization",
  "term_id": "GO:0006325",
  "gene": "UniProtKB:Q9UFC0",
  "gene_name": "Leucine-rich repeat and WD repeat-containing protein 1",
  "gene_symbol": "LRWD1"
}